{
  "gene": "UniProtKB:Q6UWN8",
  "gene_name": "Serine protease inhibitor Kazal-type 6",
  "term_label": "serine-type endopeptidase inhibitor activity",
  "gene_symbol": "SPINK6",
  "term_id": "GO:0004867"
}